{
  "term_id": "GO:0008066",
  "gene": "UniProtKB:Q8TCU5",
  "gene_symbol": "GRIN3A",
  "gene_name": "Glutamate receptor ionotropic, NMDA 3A",
  "term_label": "glutamate receptor activity"
}